phosphatidylinositol-4,5-bisphosphate sensor activity [GO:0140550] (molecular function) References: PMID:33172987 Definition: Binding to and responding, e.g. by conformational change, to changes in the cellular level of phosphatidylinositol-4,5-bisphosphate. Relationships: is a type of lipid sensor activity [GO:0106254] Also known as: phosphatidylinositol-4,5-bisphosphate sensing activity